{
  "gene": "UniProtKB:P23921",
  "gene_name": "Ribonucleoside-diphosphate reductase large subunit",
  "gene_symbol": "RRM1",
  "term_label": "ATP binding",
  "term_id": "GO:0005524"
}